{
  "term_id": "UNKNOWN:0002",
  "gene_symbol": "USH2A",
  "gene_name": "Usherin",
  "gene": "UniProtKB:O75445",
  "term_label": "Unknown biological process"
}